L-tryptophan:pyruvate aminotransferase activity [GO:0080097] (molecular function) Sources: RHEA:27586 Relationships: is a type of L-tryptophan aminotransferase activity [GO:0070529] Definition: Catalysis of the reaction: L-tryptophan + pyruvate = 3-(indol-3-yl)pyruvate + L-alanine.